negative regulation of epidermis development [GO:0045683] (biological process) Definition: Any process that stops, prevents, or reduces the frequency, rate or extent of epidermis development. Sources: GOC:go_curators Also known as: down regulation of epidermis development, down-regulation of epidermis development, downregulation of epidermis development, negative regulation of epidermal development, inhibition of epidermis development, negative regulation of hypodermis development Relationships: is a type of regulation of epidermis development [GO:0045682]; is a type of GO:0051093; negatively regulates epidermis development [GO:0008544] Subtypes: negative regulation of epidermal cell differentiation [GO:0045605]